positive regulation of auxin mediated signaling pathway [GO:0010929] (biological process) Sources: GOC:dph, GOC:tb Relationships: is a type of GO:0009967; is a type of regulation of auxin mediated signaling pathway [GO:0010928]; positively regulates auxin-activated signaling pathway [GO:0009734] Definition: Any process that increases the rate, frequency or extent of auxin mediated signaling pathway. Auxin mediated signaling pathway is the series of molecular signals generated in response to detection of auxin. Also known as: positive regulation of auxin mediated signalling pathway